{
  "gene_name": "Cholesterol 24-hydroxylase",
  "term_label": "Unknown cellular component",
  "term_id": "UNKNOWN:0003",
  "gene": "UniProtKB:Q9Y6A2",
  "gene_symbol": "CYP46A1"
}